detection of mechanical stimulus involved in sensory perception of touch [GO:0050976] (biological process) Regulation: regulated by regulation of detection of mechanical stimulus involved in sensory perception of touch [GO:1905787]; negatively regulated by negative regulation of detection of mechanical stimulus involved in sensory perception of touch [GO:1905788]; positively regulated by positive regulation of detection of mechanical stimulus involved in sensory perception of touch [GO:1905789] Sources: GOC:ai, GOC:dos Also known as: perception of touch, detection of mechanical stimulus, perception of touch, sensory detection of mechanical stimulus, perception of touch, sensory transduction of mechanical stimulus, sensory detection of mechanical stimulus during perception of touch, sensory transduction of mechanical stimulus during perception of touch, tactition, sensory detection of mechanical stimulus Definition: The series of events involved in the perception of touch in which a mechanical stimulus is received and converted into a molecular signal. Relationships: is a type of GO:0050974; is part of sensory perception of touch [GO:0050975]